{
  "gene_symbol": "ARHGAP4",
  "gene": "UniProtKB:P98171",
  "gene_name": "Rho GTPase-activating protein 4",
  "term_label": "regulation of synapse assembly",
  "term_id": "GO:0051963"
}